{
  "gene_symbol": "SHC4",
  "term_id": "GO:0005886",
  "gene_name": "SHC-transforming protein 4",
  "gene": "UniProtKB:Q6S5L8",
  "term_label": "plasma membrane"
}